{
  "gene": "UniProtKB:P01303",
  "gene_name": "Pro-neuropeptide Y",
  "gene_symbol": "NPY",
  "term_label": "neuropeptide hormone activity",
  "term_id": "GO:0005184"
}